{
  "term_label": "beta-alanine biosynthetic process via 3-ureidopropionate",
  "term_id": "GO:0033396",
  "gene_name": "Beta-ureidopropionase",
  "gene": "UniProtKB:Q9UBR1",
  "gene_symbol": "UPB1"
}